{
  "gene_symbol": "UBA52",
  "term_label": "protein ubiquitination",
  "gene_name": "Ubiquitin-ribosomal protein eL40 fusion protein",
  "term_id": "GO:0016567",
  "gene": "UniProtKB:P62987"
}